{
  "term_id": "GO:1900029",
  "gene_symbol": "EPS8",
  "term_label": "positive regulation of ruffle assembly",
  "gene_name": "Epidermal growth factor receptor kinase substrate 8",
  "gene": "UniProtKB:Q12929"
}